{
  "term_label": "choline transmembrane transporter activity",
  "term_id": "GO:0015220",
  "gene_symbol": "SLC44A1",
  "gene": "UniProtKB:Q8WWI5",
  "gene_name": "Choline transporter-like protein 1"
}